{
  "term_label": "sulfurtransferase activity",
  "term_id": "GO:0016783",
  "gene_symbol": "CTU2",
  "gene_name": "Cytoplasmic tRNA 2-thiolation protein 2",
  "gene": "UniProtKB:Q2VPK5"
}